phosphatidate-sterol O-acyltransferase activity [GO:0080096] (molecular function) Relationships: is_a O-acyltransferase activity [GO:0008374] Definition: Catalysis of the reaction: a phosphatidate + a sterol = a sterol ester + a lysophosphatidate. References: PMID:16020547